{
  "gene": "UniProtKB:Q9NZC2",
  "gene_symbol": "TREM2",
  "term_id": "GO:0045088",
  "gene_name": "Triggering receptor expressed on myeloid cells 2",
  "term_label": "regulation of innate immune response"
}